sulfolipid biosynthetic process [GO:0046506] (biological process) Definition: The chemical reactions and pathways resulting in the formation of sulfolipid, a compound containing a sulfonic acid residue joined by a carbon-sulfur bond to a lipid. Also known as: sulfolipid anabolism, sulfolipid biosynthesis, sulfolipid formation, sulfolipid synthesis, sulpholipid biosynthesis, sulpholipid biosynthetic process Relationships: is a type of lipid biosynthetic process [GO:0008610]; is a type of sulfur compound biosynthetic process [GO:0044272]; is a type of sulfolipid metabolic process [GO:0046505] References: PMID:9751667